type 2 neuropeptide Y receptor binding [GO:0031843] (molecular function) Definition: Binding to a type 2 neuropeptide Y receptor. Also known as: type 2 neuropeptide Y receptor ligand Sources: GOC:mah, GOC:nln Relationships: is a type of GO:0031841